{
  "term_id": "UNKNOWN:0002",
  "term_label": "Unknown biological process",
  "gene": "UniProtKB:Q9H1E5",
  "gene_name": "Thioredoxin-related transmembrane protein 4",
  "gene_symbol": "TMX4"
}